{
  "gene_name": "C-C motif chemokine 4",
  "gene_symbol": "CCL4",
  "term_label": "eosinophil chemotaxis",
  "term_id": "GO:0048245",
  "gene": "UniProtKB:P13236"
}